protein xylosyltransferase activity [GO:0030158] (molecular function) Also known as: peptide O-xylosyltransferase activity, UDP-D-xylose:core protein beta-D-xylosyltransferase activity, UDP-D-xylose:core protein xylosyltransferase activity, UDP-D-xylose:protein beta-D-xylosyltransferase activity, UDP-D-xylose:proteoglycan core protein beta-D-xylosyltransferase activity, UDP-xylose-core protein beta-D-xylosyltransferase activity, uridine diphosphoxylose-core protein beta-xylosyltransferase activity, uridine diphosphoxylose-protein xylosyltransferase activity Sources: EC:2.4.2.26 Relationships: is_a UDP-xylosyltransferase activity [GO:0035252]; is a type of GO:0140096 Definition: Catalysis of the transfer of a beta-D-xylosyl residue from UDP-D-xylose to the serine hydroxyl group of an acceptor protein substrate.